{
  "term_label": "GDP-L-fucose salvage",
  "gene_symbol": "FCSK",
  "gene": "UniProtKB:Q8N0W3",
  "gene_name": "L-fucose kinase",
  "term_id": "GO:0042352"
}